{
  "gene_name": "Gastrotropin",
  "term_label": "nucleus",
  "gene_symbol": "FABP6",
  "term_id": "GO:0005634",
  "gene": "UniProtKB:P51161"
}